linear polyubiquitin binding [GO:1990450] (molecular function) References: PMID:23453807 Sources: GOC:PARL, GOC:bf Relationships: is a type of GO:0043130 Definition: Binding to a linear polymer of ubiquitin. Linear ubiquitin polymers are formed by linking the amino-terminal methionine (M1) of one ubiquitin molecule to the carboxy-terminal glycine (G76) of the next. Also known as: M1-linked ubiquitin chain binding